{
  "term_id": "UNKNOWN:0003",
  "term_label": "Unknown cellular component",
  "gene_name": "HLA class I histocompatibility antigen protein P5",
  "gene_symbol": "HCP5",
  "gene": "UniProtKB:Q6MZN7"
}